{
  "gene_symbol": "CDV3",
  "term_id": "UNKNOWN:0001",
  "term_label": "Unknown molecular function",
  "gene_name": "Protein CDV3 homolog",
  "gene": "UniProtKB:Q9UKY7"
}